{
  "term_id": "GO:0000445",
  "gene_symbol": "THOC3",
  "gene": "UniProtKB:Q96J01",
  "gene_name": "THO complex subunit 3",
  "term_label": "THO complex part of transcription export complex"
}